{
  "term_label": "Unknown cellular component",
  "gene_name": "Docking protein 3",
  "gene": "UniProtKB:Q7L591",
  "term_id": "UNKNOWN:0003",
  "gene_symbol": "DOK3"
}